{
  "gene_name": "Sorting nexin-8",
  "gene": "UniProtKB:Q9Y5X2",
  "term_id": "UNKNOWN:0001",
  "term_label": "Unknown molecular function",
  "gene_symbol": "SNX8"
}